{
  "gene": "UniProtKB:Q86YH2",
  "term_label": "DNA-binding transcription factor activity, RNA polymerase II-specific",
  "term_id": "GO:0000981",
  "gene_name": "Zinc finger protein 280B",
  "gene_symbol": "ZNF280B"
}